photoreceptor outer segment [GO:0001750] (cellular component) Definition: The outer segment of a vertebrate photoreceptor that contains a stack of membrane discs embedded with photoreceptor proteins. References: PMID:19501669, PMID:26574505, PMID:6771304 Sources: GOC:cilia, GOC:krc, GOC:pde, ISBN:0824072820 Relationships: is a type of GO:0110165; is part of photoreceptor cell cilium [GO:0097733] Subtypes: cone photoreceptor outer segment [GO:0120199], GO:0120200